{
  "gene": "UniProtKB:Q93098",
  "term_id": "GO:0005125",
  "term_label": "cytokine activity",
  "gene_symbol": "WNT8B",
  "gene_name": "Protein Wnt-8b"
}